{
  "term_id": "GO:0042058",
  "gene": "UniProtKB:Q6PJF5",
  "gene_symbol": "RHBDF2",
  "gene_name": "Inactive rhomboid protein 2",
  "term_label": "regulation of epidermal growth factor receptor signaling pathway"
}